{
  "gene_symbol": "CSNK1G2",
  "gene": "UniProtKB:P78368",
  "gene_name": "Casein kinase I isoform gamma-2",
  "term_label": "endocytosis",
  "term_id": "GO:0006897"
}